{
  "term_label": "nucleus",
  "gene": "UniProtKB:Q15631",
  "gene_name": "Translin",
  "gene_symbol": "TSN",
  "term_id": "GO:0005634"
}